{
  "gene_symbol": "S100Z",
  "gene": "UniProtKB:Q8WXG8",
  "term_id": "GO:0005509",
  "term_label": "calcium ion binding",
  "gene_name": "Protein S100-Z"
}